chimeric colonial development [GO:0099135] (biological process) Definition: Development a structure consisting of multiple co-operating unicellular organisms of the same species, involving cells of more that one genotype. References: PMID:18272966 Relationships: is a type of socially cooperative development [GO:0099120] Subtypes: GO:0099136